{
  "term_id": "GO:0034109",
  "gene_name": "Coxsackievirus and adenovirus receptor",
  "gene": "UniProtKB:P78310",
  "term_label": "homotypic cell-cell adhesion",
  "gene_symbol": "CXADR"
}